{
  "gene_name": "Transcription elongation factor SPT6",
  "term_label": "nucleosome binding",
  "gene": "UniProtKB:Q7KZ85",
  "gene_symbol": "SUPT6H",
  "term_id": "GO:0031491"
}